{
  "gene": "UniProtKB:A0A2R8YEV3",
  "term_id": "UNKNOWN:0001",
  "term_label": "Unknown molecular function",
  "gene_name": "Olfactory receptor",
  "gene_symbol": "OR2A42"
}